{
  "gene_symbol": "SNX30",
  "term_label": "early endosome",
  "gene": "UniProtKB:Q5VWJ9",
  "term_id": "GO:0005769",
  "gene_name": "Sorting nexin-30"
}